{
  "gene_symbol": "PADI2",
  "gene": "UniProtKB:Q9Y2J8",
  "term_label": "histone arginine deiminase activity",
  "term_id": "GO:0140794",
  "gene_name": "Protein-arginine deiminase type-2"
}